{
  "gene_symbol": "PRELID1",
  "gene": "UniProtKB:Q9Y255",
  "gene_name": "PRELI domain-containing protein 1, mitochondrial",
  "term_id": "GO:0015914",
  "term_label": "phospholipid transport"
}